{
  "gene": "UniProtKB:Q09470",
  "term_id": "GO:0043025",
  "gene_name": "Potassium voltage-gated channel subfamily A member 1",
  "gene_symbol": "KCNA1",
  "term_label": "neuronal cell body"
}